{
  "gene_symbol": "AP3D1",
  "gene_name": "AP-3 complex subunit delta-1",
  "term_id": "UNKNOWN:0001",
  "gene": "UniProtKB:O14617",
  "term_label": "Unknown molecular function"
}